{
  "term_label": "nucleoplasm",
  "term_id": "GO:0005654",
  "gene_symbol": "HOXD4",
  "gene": "UniProtKB:P09016",
  "gene_name": "Homeobox protein Hox-D4"
}